protocatechuate 4,5-dioxygenase activity [GO:0018579] (molecular function) Also known as: protocatechuate 4,5-oxygenase activity, protocatechuate:oxygen 4,5-oxidoreductase (decyclizing), protocatechuic 4,5-dioxygenase activity, protocatechuic 4,5-oxygenase activity Sources: EC:1.13.11.8 Definition: Catalysis of the reaction: protocatechuate + O2 = 4-carboxy-2-hydroxymuconate semialdehyde. Relationships: is a type of oxidoreductase activity, acting on single donors with incorporation of molecular oxygen, incorporation of two atoms of oxygen [GO:0016702]